lamin filament [GO:0005638] (CC) Relationships: is_a intermediate filament [GO:0005882]; is part of nuclear lamina [GO:0005652] Definition: Any of a group of intermediate-filament proteins that form the fibrous matrix on the inner surface of the nuclear envelope. They are classified as lamins A, B and C. Sources: ISBN:0198547684 Also known as: type V intermediate filament